{
  "term_id": "GO:0005634",
  "term_label": "nucleus",
  "gene_name": "Catenin delta-2",
  "gene_symbol": "CTNND2",
  "gene": "UniProtKB:Q9UQB3"
}